{
  "gene": "UniProtKB:Q9BRG1",
  "gene_name": "Vacuolar protein-sorting-associated protein 25",
  "gene_symbol": "VPS25",
  "term_label": "ESCRT II complex",
  "term_id": "GO:0000814"
}